thymine dioxygenase activity [GO:0050341] (molecular function) Also known as: 5-hydroxy-methyluracil dioxygenase activity, 5-hydroxymethyluracil oxygenase activity, thymine 7-hydroxylase activity, thymine,2-oxoglutarate dioxygenase activity, thymine,2-oxoglutarate:oxygen oxidoreductase (7-hydroxylating) Sources: EC:1.14.11.6, MetaCyc:THYMINE-DIOXYGENASE-RXN Relationships: is a type of 2-oxoglutarate-dependent dioxygenase activity [GO:0016706] Definition: Catalysis of the reaction: thymine + 2-oxoglutarate + O2 = 5-hydroxymethyluracil + succinate + CO2.